{
  "gene_name": "Transmembrane protein 107",
  "gene": "UniProtKB:Q6UX40",
  "term_id": "GO:0036038",
  "term_label": "MKS complex",
  "gene_symbol": "TMEM107"
}